{
  "term_id": "UNKNOWN:0001",
  "gene_symbol": "LUZP1",
  "gene_name": "Leucine zipper protein 1",
  "gene": "UniProtKB:Q86V48",
  "term_label": "Unknown molecular function"
}